{
  "gene": "UniProtKB:P33176",
  "gene_symbol": "KIF5B",
  "term_label": "cytoplasm",
  "term_id": "GO:0005737",
  "gene_name": "Kinesin-1 heavy chain"
}